{
  "term_id": "GO:0006631",
  "gene_name": "Acyl-CoA-binding domain-containing protein 7",
  "gene_symbol": "ACBD7",
  "gene": "UniProtKB:Q8N6N7",
  "term_label": "fatty acid metabolic process"
}